early recombination nodule [GO:0005714] (cellular component) Definition: An electron dense structure that is associated with meiotic chromosomes in leptotene or zygotene during meiosis I. Relationships: is a type of recombination nodule [GO:0005713] Sources: GOC:elh